{
  "term_label": "fatty acid transport",
  "gene_name": "Fatty acid-binding protein, intestinal",
  "gene": "UniProtKB:P12104",
  "term_id": "GO:0015908",
  "gene_symbol": "FABP2"
}